{
  "gene": "UniProtKB:Q8WWZ4",
  "gene_name": "ATP-binding cassette sub-family A member 10",
  "term_label": "ATPase-coupled transmembrane transporter activity",
  "gene_symbol": "ABCA10",
  "term_id": "GO:0042626"
}